protein-N-terminal asparagine amidohydrolase activity [GO:0008418] (molecular function) Definition: Catalysis of the reaction: N-terminal L-asparaginyl-[protein] + H+ + H2O = N-terminal L-aspartyl-[protein] + NH4+. This reaction is the deamidation of an N-terminal asparagine residue in a peptide or protein. References: PMID:8910481 Sources: RHEA:50676 Relationships: is a type of protein asparagine deamidase activity [GO:0160260]